{
  "term_id": "GO:0007155",
  "gene": "UniProtKB:A6NMY6",
  "gene_symbol": "ANXA2P2",
  "term_label": "cell adhesion",
  "gene_name": "Putative annexin A2-like protein"
}